endocardial cushion cell fate commitment [GO:0061445] (biological process) Definition: The commitment of a cell to an endocardial cushion cell fate and its capacity to differentiate into an endocardial cushion cell. Relationships: is a type of endocardial cell fate commitment [GO:0060957]; is part of GO:0061443 Sources: GOC:BHF, GOC:dph